negative regulation of neuron projection arborization [GO:0150013] (biological process) Definition: Any process that stops, prevents or reduces the frequency, rate or extent of the process in which the anatomical structures of a neuron projection are generated and organized into branches. References: PMID:17114044 Sources: GOC:aruk, GOC:bc Also known as: negative regulation of neurite arborization, negative regulation of neurite branching, negative regulation of neuron projection branching Relationships: is_a negative regulation of cell projection organization [GO:0031345]; is a type of GO:0051093; is a type of GO:0150011; negatively regulates neuron projection arborization [GO:0140058]